{
  "gene_name": "Zinc finger protein 74",
  "term_label": "nucleus",
  "gene_symbol": "ZNF74",
  "term_id": "GO:0005634",
  "gene": "UniProtKB:Q16587"
}